{
  "gene_name": "Nuclear distribution protein nudE homolog 1",
  "gene": "UniProtKB:Q9NXR1",
  "term_label": "kinesin complex",
  "gene_symbol": "NDE1",
  "term_id": "GO:0005871"
}